{
  "gene_name": "Protein FAM131B",
  "term_id": "UNKNOWN:0001",
  "gene": "UniProtKB:Q86XD5",
  "gene_symbol": "FAM131B",
  "term_label": "Unknown molecular function"
}